{
  "term_id": "GO:0007173",
  "gene_name": "Protransforming growth factor alpha",
  "gene": "UniProtKB:P01135",
  "term_label": "epidermal growth factor receptor signaling pathway",
  "gene_symbol": "TGFA"
}